{
  "gene_name": "Nitric oxide synthase 1",
  "term_label": "L-arginine catabolic process",
  "term_id": "GO:0006527",
  "gene_symbol": "NOS1",
  "gene": "UniProtKB:P29475"
}